{
  "gene_name": "Histamine N-methyltransferase",
  "term_id": "UNKNOWN:0002",
  "gene": "UniProtKB:P50135",
  "term_label": "Unknown biological process",
  "gene_symbol": "HNMT"
}